{
  "term_label": "endocytic vesicle",
  "gene_name": "Ras-related protein Rab-24",
  "gene": "UniProtKB:Q969Q5",
  "term_id": "GO:0030139",
  "gene_symbol": "RAB24"
}